positive regulation of multicellular organismal process [GO:0051240] (biological process) Definition: Any process that activates or increases the frequency, rate or extent of an organismal process, any of the processes pertinent to the function of an organism above the cellular level; includes the integrated processes of tissues and organs. Sources: GOC:ai Also known as: up regulation of multicellular organismal process, up-regulation of multicellular organismal process, upregulation of multicellular organismal process, activation of multicellular organismal process, stimulation of multicellular organismal process Relationships: is a type of positive regulation of biological process [GO:0048518]; is_a regulation of multicellular organismal process [GO:0051239]; positively regulates GO:0032501 Subtypes: positive regulation of cytokine production [GO:0001819], positive regulation of tolerance induction [GO:0002645], positive regulation of glomerular filtration [GO:0003104], GO:0010718, positive regulation of very-low-density lipoprotein particle remodeling [GO:0010902], positive regulation of lipoprotein particle clearance [GO:0010986], positive regulation of muscle hypertrophy [GO:0014742], GO:0014744, GO:0031646, positive regulation of heat generation [GO:0031652], positive regulation of heat dissipation [GO:0031656], positive regulation of gonadotropin secretion [GO:0032278], positive regulation of neurotrophin production [GO:0032901], positive regulation of mammary gland epithelial cell proliferation [GO:0033601], positive regulation of tissue remodeling [GO:0034105], positive regulation of leukotriene production involved in inflammatory response [GO:0035491], positive regulation of renal sodium excretion [GO:0035815], positive regulation of multicellular organism growth [GO:0040018], positive regulation of embryonic development [GO:0040019], positive regulation of hair cycle [GO:0042635], positive regulation of keratinocyte differentiation [GO:0045618], GO:0045690, positive regulation of embryo sac central cell differentiation [GO:0045693], GO:0045696, positive regulation of synergid differentiation [GO:0045699], positive regulation of salivary gland boundary specification [GO:0045706], positive regulation of ossification [GO:0045778], GO:0045780, positive regulation of chitin-based cuticle tanning [GO:0045801], positive regulation of eclosion [GO:0045805], positive regulation of vasoconstriction [GO:0045907], positive regulation of muscle contraction [GO:0045933], GO:0046534, positive regulation of organ growth [GO:0046622], positive regulation of cuticle pigmentation [GO:0048081], positive regulation of female pigmentation [GO:0048091], GO:0048093, positive regulation of behavior [GO:0048520], positive regulation of post-embryonic development [GO:0048582], GO:0048636, positive regulation of coagulation [GO:0050820], positive regulation of cell activation [GO:0050867], positive regulation of corticotropin secretion [GO:0051461], positive regulation of hair follicle development [GO:0051798], positive regulation of nervous system development [GO:0051962], positive regulation of respiratory burst involved in inflammatory response [GO:0060265], positive regulation of ovulation [GO:0060279], positive regulation of penile erection [GO:0060406], positive regulation of digestive system process [GO:0060456], positive regulation of mammary placode formation by mesenchymal-epithelial signaling [GO:0060617], positive regulation of cartilage development [GO:0061036], positive regulation of branching involved in lung morphogenesis [GO:0061047], positive regulation of cardiac endothelial to mesenchymal transition [GO:0062000], positive regulation of adiponectin secretion [GO:0070165], positive regulation of mucus secretion [GO:0070257], positive regulation of hepatocyte differentiation [GO:0070368], positive regulation of spore-bearing organ development [GO:0075261], GO:0090108, positive regulation of kidney development [GO:0090184], positive regulation of branching involved in ureteric bud morphogenesis [GO:0090190], positive regulation of chylomicron remodeling [GO:0090319], positive regulation of pupariation [GO:0106025], GO:0110039, positive regulation of imaginal disc-derived wing vein specification [GO:0110108], positive regulation of animal organ morphogenesis [GO:0110110], positive regulation of cold-induced thermogenesis [GO:0120162], positive regulation of adenylate cyclase-activating adrenergic receptor signaling pathway involved in heart process [GO:0140196], positive regulation of transport across blood-brain barrier [GO:0150201], positive regulation of amyloid-beta clearance [GO:1900223], GO:1901079, positive regulation of trophoblast cell migration [GO:1901165], positive regulation of lung ciliated cell differentiation [GO:1901248], GO:1901251, positive regulation of seed dormancy process [GO:1902040], GO:1902459, positive regulation of sperm capacitation [GO:1902492], positive regulation of lens fiber cell differentiation [GO:1902748], positive regulation of renal amino acid absorption [GO:1902754], positive regulation of retina development in camera-type eye [GO:1902868], GO:1902877, positive regulation of bone development [GO:1903012], positive regulation of vitellogenesis [GO:1903188], GO:1903367, positive regulation of renal phosphate excretion [GO:1903404], positive regulation of lactation [GO:1903489], positive regulation of blood circulation [GO:1903524], positive regulation of histamine secretion by mast cell [GO:1903595], positive regulation of epithelial cell-cell adhesion involved in epithelium migration [GO:1903683], positive regulation of hemopoiesis [GO:1903708], positive regulation of collecting lymphatic vessel constriction [GO:1903816], positive regulation of respiratory gaseous exchange [GO:1903942], GO:1904018, positive regulation of adipose tissue development [GO:1904179], positive regulation of transcytosis [GO:1904300], positive regulation of maternal process involved in parturition [GO:1904303], positive regulation of cardiac ventricle development [GO:1904414], positive regulation of thyroid gland epithelial cell proliferation [GO:1904443], positive regulation of lung alveolus development [GO:1904655], positive regulation of male germ-line stem cell asymmetric division [GO:1904840], positive regulation of apical ectodermal ridge formation [GO:1905142], positive regulation of cardiocyte differentiation [GO:1905209], positive regulation of epithelial tube formation [GO:1905278], positive regulation of epidermal growth factor receptor signaling pathway involved in heart process [GO:1905284], GO:1905294, positive regulation of intestinal epithelial cell development [GO:1905300], positive regulation of plant organ morphogenesis [GO:1905423], GO:1905492, GO:1905623, positive regulation of oogenesis [GO:1905881], positive regulation of germ cell proliferation [GO:1905938], GO:1905941, positive regulation of endothelial tube morphogenesis [GO:1905956], positive regulation of determination of dorsal identity [GO:2000017], positive regulation of ureter smooth muscle cell differentiation [GO:2000063], GO:2000078, GO:2000103, positive regulation of pancreatic A cell differentiation [GO:2000228], positive regulation of fibroblast growth factor receptor signaling pathway involved in neural plate anterior/posterior pattern formation [GO:2000315], positive regulation of renal albumin absorption [GO:2000534], GO:2000693, positive regulation of mesenchymal cell proliferation involved in lung development [GO:2000792], positive regulation of parathyroid hormone secretion [GO:2000830], positive regulation of steroid hormone secretion [GO:2000833], GO:2001153